{
  "term_id": "GO:0005737",
  "gene_symbol": "CFL2",
  "term_label": "cytoplasm",
  "gene_name": "Cofilin-2",
  "gene": "UniProtKB:Q9Y281"
}